{
  "gene_symbol": "TUBA4A",
  "gene_name": "Tubulin alpha-4A chain",
  "gene": "UniProtKB:P68366",
  "term_id": "GO:0005874",
  "term_label": "microtubule"
}